{
  "term_id": "GO:0032922",
  "gene": "UniProtKB:Q7Z5J4",
  "term_label": "circadian regulation of gene expression",
  "gene_name": "Retinoic acid-induced protein 1",
  "gene_symbol": "RAI1"
}